{
  "gene": "UniProtKB:Q5JQC9",
  "term_label": "cell surface receptor protein serine/threonine kinase signaling pathway",
  "gene_name": "A-kinase anchor protein 4",
  "term_id": "GO:0007178",
  "gene_symbol": "AKAP4"
}